regulation of translational initiation by eIF2 alpha dephosphorylation [GO:0036496] (biological process) Definition: Any process that modulates the frequency, rate or extent of translation initiation in response to stress by the dephosphorylation of eIF2 alpha. Subtypes: eIF2alpha dephosphorylation in response to endoplasmic reticulum stress [GO:0036497] Relationships: is a type of protein dephosphorylation [GO:0006470]; is a type of regulation of cellular component size [GO:0032535]; is a type of regulation of translational initiation in response to stress [GO:0043558] Sources: GOC:PARL, GOC:bf